DNA helicase complex [GO:0033202] (cellular component) Relationships: is a type of catalytic complex [GO:1902494] Definition: A protein complex that possesses DNA helicase activity. Subtypes: Holliday junction helicase complex [GO:0009379], single-stranded DNA-dependent ATP-dependent DNA helicase complex [GO:0017117], GO:0031422, DNA helicase A complex [GO:0033203], GO:0034980, FHL3-CREB complex [GO:0034981], DnaB-DnaG complex [GO:1990156], DnaB helicase complex [GO:1990161] Sources: GOC:mah